{
  "gene_symbol": "DAB2IP",
  "term_label": "GTPase activator activity",
  "gene_name": "Disabled homolog 2-interacting protein",
  "term_id": "GO:0005096",
  "gene": "UniProtKB:Q5VWQ8"
}